{
  "gene_symbol": "DUSP3",
  "term_id": "GO:0050860",
  "term_label": "negative regulation of T cell receptor signaling pathway",
  "gene_name": "Dual specificity protein phosphatase 3",
  "gene": "UniProtKB:P51452"
}